{
  "term_label": "cell surface receptor protein tyrosine kinase signaling pathway",
  "gene_symbol": "TIE1",
  "term_id": "GO:0007169",
  "gene": "UniProtKB:P35590",
  "gene_name": "Tyrosine-protein kinase receptor Tie-1"
}